toll-like receptor 11 signaling pathway [GO:0034170] (biological process) Regulation: regulated by GO:0034171; negatively regulated by GO:0034172; positively regulated by positive regulation of toll-like receptor 11 signaling pathway [GO:0034173] Relationships: is a type of endolysosomal toll-like receptor signaling pathway [GO:0140894] Definition: The series of molecular signals initiated by a ligand binding to the endolysosomal toll-like receptor 11. Also known as: TLR11 signaling pathway, toll-like receptor 11 signalling pathway References: PMID:16551253, PMID:17328678 Sources: GOC:add